myristoyltransferase activity [GO:0019107] (molecular function) Sources: GOC:ai Subtypes: glycylpeptide N-tetradecanoyltransferase activity [GO:0004379], peptidyl-lysine N6-myristoyltransferase activity [GO:0018030], protein-cysteine S-myristoyltransferase activity [GO:0019705], GO:0050633 Definition: Catalysis of the transfer of a myristoyl (CH3-[CH2]12-CO-) group to an acceptor molecule. Relationships: is a type of acyltransferase activity, transferring groups other than amino-acyl groups [GO:0016747]